{
  "gene_symbol": "ABCA9",
  "term_label": "lipid transporter activity",
  "term_id": "GO:0005319",
  "gene": "UniProtKB:Q8IUA7",
  "gene_name": "ATP-binding cassette sub-family A member 9"
}